regulation of convergent extension involved in axis elongation [GO:1901232] (biological process) Relationships: is a type of GO:0048638; is a type of GO:1905330; regulates convergent extension involved in axis elongation [GO:0060028] Subtypes: negative regulation of convergent extension involved in axis elongation [GO:1901233], GO:1901234, regulation of convergent extension involved in somitogenesis [GO:1904127] Definition: Any process that modulates the frequency, rate or extent of convergent extension involved in axis elongation. Sources: GOC:BHF, GOC:TermGenie